{
  "term_label": "spermatid development",
  "gene_name": "Protein FAM9C",
  "gene_symbol": "FAM9C",
  "gene": "UniProtKB:Q8IZT9",
  "term_id": "GO:0007286"
}